{
  "term_id": "GO:0031838",
  "gene": "UniProtKB:Q6B0K9",
  "gene_symbol": "HBM",
  "term_label": "haptoglobin-hemoglobin complex",
  "gene_name": "Hemoglobin subunit mu"
}